{
  "gene_name": "Probable G-protein coupled receptor 173",
  "gene": "UniProtKB:Q9NS66",
  "term_id": "UNKNOWN:0002",
  "gene_symbol": "GPR173",
  "term_label": "Unknown biological process"
}